{
  "term_label": "regulation of transcription by RNA polymerase II",
  "gene_name": "Zinc finger protein 410",
  "term_id": "GO:0006357",
  "gene": "UniProtKB:Q86VK4",
  "gene_symbol": "ZNF410"
}